{
  "term_label": "RNA polymerase II cis-regulatory region sequence-specific DNA binding",
  "gene_name": "Paired-like homeodomain transcription factor LEUTX",
  "gene_symbol": "LEUTX",
  "gene": "UniProtKB:A8MZ59",
  "term_id": "GO:0000978"
}